{
  "gene_name": "Atrial natriuretic peptide receptor 3",
  "gene": "UniProtKB:P17342",
  "gene_symbol": "NPR3",
  "term_label": "signal transduction",
  "term_id": "GO:0007165"
}